{
  "gene_name": "Tyrosine-protein kinase Blk",
  "term_id": "GO:0007169",
  "gene_symbol": "BLK",
  "gene": "UniProtKB:P51451",
  "term_label": "cell surface receptor protein tyrosine kinase signaling pathway"
}